{
  "gene_name": "DNA-directed RNA polymerase II subunit RPB11-b2",
  "term_label": "transcription by RNA polymerase II",
  "gene_symbol": "POLR2J3",
  "gene": "UniProtKB:Q9H1A7",
  "term_id": "GO:0006366"
}